trisporic acid biosynthetic process [GO:0046842] (biological process) Also known as: trisporic acid anabolism, trisporic acid biosynthesis, trisporic acid formation, trisporic acid synthesis Sources: GOC:ai Definition: The chemical reactions and pathways resulting in the formation of trisporic acid. Relationships: is_a terpenoid biosynthetic process [GO:0016114]